{
  "gene_symbol": "DQX1",
  "gene": "UniProtKB:Q8TE96",
  "gene_name": "ATP-dependent RNA helicase DQX1",
  "term_id": "UNKNOWN:0002",
  "term_label": "Unknown biological process"
}